{
  "gene_symbol": "PRTG",
  "gene_name": "Protogenin",
  "term_id": "GO:0098609",
  "gene": "UniProtKB:Q2VWP7",
  "term_label": "cell-cell adhesion"
}